{
  "gene_name": "Sorting nexin-33",
  "term_label": "endosomal transport",
  "term_id": "GO:0016197",
  "gene": "UniProtKB:Q8WV41",
  "gene_symbol": "SNX33"
}